{
  "term_label": "sarcolemma",
  "term_id": "GO:0042383",
  "gene_symbol": "ANXA8L1",
  "gene": "UniProtKB:Q5VT79",
  "gene_name": "Annexin A8-like protein 1"
}